{
  "term_id": "GO:0031012",
  "gene_symbol": "OPTC",
  "gene": "UniProtKB:Q9UBM4",
  "gene_name": "Opticin",
  "term_label": "extracellular matrix"
}